{
  "gene_symbol": "MBD3L3",
  "term_id": "GO:0005634",
  "gene": "UniProtKB:A6NE82",
  "term_label": "nucleus",
  "gene_name": "Putative methyl-CpG-binding domain protein 3-like 3"
}